{
  "term_label": "cell-cell adhesion mediated by cadherin",
  "term_id": "GO:0044331",
  "gene": "UniProtKB:Q14517",
  "gene_name": "Protocadherin Fat 1",
  "gene_symbol": "FAT1"
}